{
  "term_id": "GO:0005814",
  "term_label": "centriole",
  "gene_symbol": "HYLS1",
  "gene_name": "Centriolar and ciliogenesis-associated protein HYLS1",
  "gene": "UniProtKB:Q96M11"
}